{
  "term_label": "action potential",
  "term_id": "GO:0001508",
  "gene_symbol": "KCNG4",
  "gene_name": "Potassium voltage-gated channel subfamily G member 4",
  "gene": "UniProtKB:Q8TDN1"
}